positive regulation of leaf development [GO:1905623] (biological process) References: PMID:11606552 Sources: GOC:TermGenie, GO_REF:0000058 Definition: Any process that activates or increases the frequency, rate or extent of leaf development. Relationships: is a type of positive regulation of developmental process [GO:0051094]; is a type of positive regulation of multicellular organismal process [GO:0051240]; is_a GO:2000024; positively regulates leaf development [GO:0048366] Also known as: up regulation of leaf development, up-regulation of leaf development, upregulation of leaf development, activation of leaf development Subtypes: positive regulation of leaflet formation by auxin mediated signaling pathway [GO:0090015]